{
  "term_label": "transmembrane transporter binding",
  "gene_symbol": "SCN3B",
  "gene": "UniProtKB:Q9NY72",
  "gene_name": "Sodium channel subunit beta-3",
  "term_id": "GO:0044325"
}